{
  "gene": "UniProtKB:Q15796",
  "gene_name": "Mothers against decapentaplegic homolog 2",
  "term_id": "GO:0000978",
  "term_label": "RNA polymerase II cis-regulatory region sequence-specific DNA binding",
  "gene_symbol": "SMAD2"
}